NLS-dependent protein nuclear import complex [GO:0042564] (CC) References: PMID:9323123, PMID:9323134 Sources: GOC:jl, Wikipedia:Importin Relationships: is a type of nucleocytoplasmic transport complex [GO:0031074] Definition: A dimer consisting of an alpha and a beta-subunit that imports proteins with an NLS into the nucleus through a nuclear pore.